histone H2AXY142 kinase activity [GO:0140801] (molecular function) Definition: Catalysis of the reaction: histone H2AX-tyrosine (position 142) + ATP = (histone H2AX-phosphotyrosine (position 142) + ADP. This reaction is the addition of a phosphate group to the serine residue at position 142 of histone variant H2AX. References: PMID:19092802 Note: Note that the residue position corresponds to the canonical human H2AX histone (UniProtKB:P16104); this residue is conserved in mammals, but missing from tetrahymena. This residue is present in Drosophila histone H2AV. Residue 1 is the first residue following removal of the initiating Methionine (Met). Note that each histone is encoded by multiple genes, and sequences may vary across different genes within an organism. Also known as: gamma-H2AX-S142 kinase activity, histone H2AX-Y142 kinase activity, histone kinase activity (H2AX-Y142 specific), histone H2AY142 kinase activity Relationships: is a type of protein tyrosine kinase activity [GO:0004713]; is_a histone H2AX kinase activity [GO:0141003]